{
  "gene_symbol": "ZG16",
  "term_label": "Unknown molecular function",
  "gene": "UniProtKB:O60844",
  "gene_name": "Zymogen granule membrane protein 16",
  "term_id": "UNKNOWN:0001"
}